NAD+ metabolic process [GO:0019674] (biological process) Subtypes: glycerol-3-phosphate shuttle [GO:0006127], NADH regeneration [GO:0006735], NAD+ biosynthetic process [GO:0009435], NAD+ catabolic process [GO:0019677], GO:0043490 Relationships: is a type of purine nucleotide metabolic process [GO:0006163]; is a type of nicotinamide nucleotide metabolic process [GO:0046496] Also known as: NAD (oxidized) metabolic process, NAD (oxidized) metabolism, NAD metabolic process, NAD metabolism, nicotinamide adenine dinucleotide metabolic process, nicotinamide adenine dinucleotide metabolism, oxidized NAD metabolic process, oxidized NAD metabolism, oxidized nicotinamide adenine dinucleotide metabolic process, oxidized nicotinamide adenine dinucleotide metabolism, NAD phosphorylation and dephosphorylation References: PMID:28648096 Regulation: regulated by regulation of NAD metabolic process [GO:1902688]; RO_0002212 by negative regulation of NAD metabolic process [GO:1902689]; positively regulated by GO:1902690 Definition: The chemical reactions and pathways involving nicotinamide adenine dinucleotide (NAD+), a coenzyme that interconverts with its reduced form, NADH, in many redox and catabolic reactions.